{
  "term_id": "GO:1990756",
  "gene": "UniProtKB:Q99619",
  "gene_name": "SPRY domain-containing SOCS box protein 2",
  "gene_symbol": "SPSB2",
  "term_label": "ubiquitin-like ligase-substrate adaptor activity"
}